{
  "gene_name": "NKG2-A_NKG2-B type II integral membrane protein",
  "term_id": "GO:0002228",
  "gene": "UniProtKB:P26715",
  "gene_symbol": "KLRC1",
  "term_label": "natural killer cell mediated immunity"
}